{
  "gene_name": "Acyl-CoA wax alcohol acyltransferase 1",
  "term_id": "GO:0047196",
  "gene": "UniProtKB:Q58HT5",
  "gene_symbol": "AWAT1",
  "term_label": "long-chain-alcohol O-fatty-acyltransferase activity"
}